{
  "gene": "UniProtKB:Q8N4N8",
  "gene_name": "Kinesin-like protein KIF2B",
  "term_label": "microtubule binding",
  "term_id": "GO:0008017",
  "gene_symbol": "KIF2B"
}